{
  "gene": "UniProtKB:O14684",
  "gene_symbol": "PTGES",
  "term_label": "membrane",
  "gene_name": "Prostaglandin E synthase",
  "term_id": "GO:0016020"
}